{
  "term_label": "dendrite",
  "gene_symbol": "HCN1",
  "gene": "UniProtKB:O60741",
  "term_id": "GO:0030425",
  "gene_name": "Potassium_sodium hyperpolarization-activated cyclic nucleotide-gated channel 1"
}